{
  "term_label": "protein serine/threonine kinase activity",
  "term_id": "GO:0004674",
  "gene_name": "Serine_threonine-protein kinase PAK 6",
  "gene": "UniProtKB:Q9NQU5",
  "gene_symbol": "PAK6"
}